{
  "term_label": "G protein-coupled peptide receptor activity",
  "term_id": "GO:0008528",
  "gene_symbol": "GIPR",
  "gene": "UniProtKB:P48546",
  "gene_name": "Gastric inhibitory polypeptide receptor"
}